{
  "gene_symbol": "DYNLT5",
  "term_id": "GO:0005737",
  "gene_name": "Dynein light chain Tctex-type 5",
  "gene": "UniProtKB:Q8N7M0",
  "term_label": "cytoplasm"
}